{
  "gene": "UniProtKB:Q5GLZ8",
  "term_id": "GO:0005737",
  "gene_name": "Probable E3 ubiquitin-protein ligase HERC4",
  "term_label": "cytoplasm",
  "gene_symbol": "HERC4"
}